{
  "gene_symbol": "ADIPOQ",
  "term_label": "Unknown cellular component",
  "term_id": "UNKNOWN:0003",
  "gene_name": "Adiponectin",
  "gene": "UniProtKB:Q15848"
}